{
  "term_label": "synapse",
  "term_id": "GO:0045202",
  "gene_name": "Exocyst complex component 4",
  "gene": "UniProtKB:Q96A65",
  "gene_symbol": "EXOC4"
}